meiotic chromosome condensation [GO:0010032] (biological process) Relationships: is a type of chromosome condensation [GO:0030261]; is a type of chromosome organization involved in meiotic cell cycle [GO:0070192] Definition: Compaction of chromatin structure prior to meiosis in eukaryotic cells. Also known as: chromosome condensation involved in meiotic cell cycle References: PMID:10072401